{
  "term_label": "nucleus",
  "term_id": "GO:0005634",
  "gene_name": "Zinc finger X-linked protein ZXDA",
  "gene": "UniProtKB:P98168",
  "gene_symbol": "ZXDA"
}